CXCR1 chemokine receptor binding [GO:0045237] (molecular function) References: PMID:11910892 Sources: GOC:ceb Definition: Binding to a CXCR1 chemokine receptor. Relationships: is a type of GO:0005153 Also known as: CXCR1 chemokine receptor ligand